nicotinate dehydrogenase activity [GO:0050138] (molecular function) Definition: Catalysis of the reaction: H2O + NADP+ + nicotinate = 6-hydroxynicotinate + H+ + NADPH. Sources: EC:1.17.1.5, RHEA:12236 Also known as: nicotinate hydroxylase activity, nicotinate:NADP+ 6-oxidoreductase (hydroxylating), nicotinic acid hydroxylase activity Relationships: is a type of GO:0016726